{
  "term_id": "GO:0005788",
  "gene_name": "Endoplasmic reticulum aminopeptidase 2",
  "gene": "UniProtKB:Q6P179",
  "gene_symbol": "ERAP2",
  "term_label": "endoplasmic reticulum lumen"
}